{
  "gene_symbol": "ATXN8OS",
  "gene_name": "Putative protein ATXN8OS",
  "term_id": "UNKNOWN:0001",
  "gene": "UniProtKB:P0DMR3",
  "term_label": "Unknown molecular function"
}